{
  "gene_symbol": "EMID1",
  "term_label": "Unknown biological process",
  "gene_name": "EMI domain-containing protein 1",
  "gene": "UniProtKB:Q96A84",
  "term_id": "UNKNOWN:0002"
}